{
  "term_label": "miRNA-mediated post-transcriptional gene silencing",
  "term_id": "GO:0035195",
  "gene_symbol": "TNRC6A",
  "gene_name": "Trinucleotide repeat-containing gene 6A protein",
  "gene": "UniProtKB:Q8NDV7"
}